host cell nuclear membrane [GO:0044200] (cellular component) Relationships: is_a host cell membrane [GO:0033644]; is part of host cell nuclear envelope [GO:0044199] Sources: GOC:jl Definition: Either of the lipid bilayers that surround the host nucleus and form the nuclear envelope; excludes the intermembrane space. Subtypes: host cell nuclear inner membrane [GO:0044201], host cell nuclear outer membrane [GO:0044202]